{
  "term_label": "DNA-binding transcription factor activity, RNA polymerase II-specific",
  "term_id": "GO:0000981",
  "gene_name": "Mothers against decapentaplegic homolog 2",
  "gene_symbol": "SMAD2",
  "gene": "UniProtKB:Q15796"
}